{
  "term_label": "extracellular space",
  "gene": "UniProtKB:P26927",
  "gene_symbol": "MST1",
  "gene_name": "Hepatocyte growth factor-like protein",
  "term_id": "GO:0005615"
}